{
  "term_id": "GO:0019814",
  "gene_name": "Probable non-functional immunoglobulin lambda variable 2-33",
  "gene": "UniProtKB:A0A075B6J2",
  "gene_symbol": "IGLV2-33",
  "term_label": "immunoglobulin complex"
}